{
  "term_label": "transcription cis-regulatory region binding",
  "gene": "UniProtKB:Q96K83",
  "term_id": "GO:0000976",
  "gene_name": "Zinc finger protein 521",
  "gene_symbol": "ZNF521"
}